{
  "term_label": "Unknown cellular component",
  "gene_name": "tRNA-specific adenosine deaminase 1",
  "gene_symbol": "ADAT1",
  "gene": "UniProtKB:Q9BUB4",
  "term_id": "UNKNOWN:0003"
}